{
  "term_id": "GO:0008201",
  "gene_name": "Interphotoreceptor matrix proteoglycan 2",
  "term_label": "heparin binding",
  "gene": "UniProtKB:Q9BZV3",
  "gene_symbol": "IMPG2"
}